{
  "gene": "UniProtKB:Q96B45",
  "gene_symbol": "BORCS7",
  "gene_name": "BLOC-1-related complex subunit 7",
  "term_id": "GO:0099078",
  "term_label": "BORC complex"
}